{
  "gene": "UniProtKB:Q9NX07",
  "gene_symbol": "TRNAU1AP",
  "term_id": "GO:0000049",
  "term_label": "tRNA binding",
  "gene_name": "tRNA selenocysteine 1-associated protein 1"
}